{
  "term_label": "nucleus",
  "term_id": "GO:0005634",
  "gene": "UniProtKB:Q8TDG4",
  "gene_name": "Helicase POLQ-like",
  "gene_symbol": "HELQ"
}